cortical Lewy body [GO:0097415] (cellular component) Definition: Cytoplasmic inclusion similar to a classical Lewy body but lacking a halo of protein fibrils. Sources: NIF_Subcellular:sao4040591221 Relationships: is a type of Lewy body [GO:0097413]